maltohexaose transport [GO:2001103] (biological process) Sources: GOC:mengo_curators Relationships: is a type of hexasaccharide transport [GO:2001102] Definition: The directed movement of a maltohexaoseacetate into, out of or within a cell, or between cells, by means of some agent such as a transporter or pore. Regulation: regulated by regulation of maltohexaose transport [GO:1900312]; negatively regulated by negative regulation of maltohexaose transport [GO:1900313]; positively regulated by positive regulation of maltohexaose transport [GO:1900314]